{
  "term_label": "chromosome segregation",
  "gene_name": "Baculoviral IAP repeat-containing protein 5",
  "gene_symbol": "BIRC5",
  "gene": "UniProtKB:O15392",
  "term_id": "GO:0007059"
}